{
  "term_id": "GO:0002128",
  "gene": "UniProtKB:Q6YHU6",
  "gene_name": "Thyroid adenoma-associated protein",
  "gene_symbol": "THADA",
  "term_label": "tRNA nucleoside ribose methylation"
}